{
  "gene_name": "Zinc finger and BTB domain-containing protein 18",
  "gene_symbol": "ZBTB18",
  "gene": "UniProtKB:Q99592",
  "term_id": "GO:0000981",
  "term_label": "DNA-binding transcription factor activity, RNA polymerase II-specific"
}